positive regulation of mesenchymal cell apoptotic process involved in mesonephric nephron morphogenesis [GO:0061297] (biological process) Sources: GOC:mtg_apoptosis, GOC:mtg_kidney_jan10 Also known as: positive regulation of mesenchymal stem cell apoptotic process involved in mesonephric nephron morphogenesis, positive regulation of mesenchymal stem cell apoptosis involved in mesonephric nephron morphogenesis Definition: Any process that increases the occurrence or rate of mesenchymal stem cell death by apoptotic process that contributes to the shaping of the nephron in the mesonephros. Relationships: is a type of positive regulation of mesonephros development [GO:0061213]; is_a GO:0061295; is a type of GO:0072041; RO_0002213 mesenchymal stem cell maintenance involved in mesonephric nephron morphogenesis [GO:0061235]; positively regulates mesenchymal cell apoptotic process involved in mesonephric nephron morphogenesis [GO:1901146]